{
  "gene_name": "cAMP-specific 3',5'-cyclic phosphodiesterase 4C",
  "term_label": "negative regulation of cAMP/PKA signal transduction",
  "term_id": "GO:0141162",
  "gene": "UniProtKB:Q08493",
  "gene_symbol": "PDE4C"
}